negative regulation of growth factor dependent skeletal muscle satellite cell proliferation [GO:1902727] (biological process) Definition: Any process that stops, prevents or reduces the frequency, rate or extent of satellite cell proliferation; dependent on specific growth factor activity such as fibroblast growth factors and transforming growth factor beta. References: PMID:23212449 Sources: GOC:TermGenie, GO_REF:0000058 Relationships: is a type of negative regulation of skeletal muscle satellite cell proliferation [GO:1902723]